negative regulation of tube lumen cavitation [GO:1903133] (biological process) Relationships: is_a negative regulation of developmental process [GO:0051093]; is a type of GO:0051241; is a type of regulation of tube lumen cavitation [GO:1903132]; negatively regulates tube lumen cavitation [GO:0060605] Also known as: inhibition of tube lumen cavitation Definition: Any process that stops, prevents or reduces the frequency, rate or extent of tube lumen cavitation. References: PMID:22898778 Sources: GOC:TermGenie, GOC:dph, GO_REF:0000058